{
  "term_id": "UNKNOWN:0001",
  "gene_symbol": "SIGMAR1",
  "term_label": "Unknown molecular function",
  "gene": "UniProtKB:Q99720",
  "gene_name": "Sigma non-opioid intracellular receptor 1"
}